positive regulation of heterotypic cell-cell adhesion [GO:0034116] (biological process) Relationships: is a type of positive regulation of cell-cell adhesion [GO:0022409]; is a type of GO:0034114; positively regulates heterotypic cell-cell adhesion [GO:0034113] Sources: GOC:add Definition: Any process that activates or increases the frequency, rate, or extent of heterotypic cell-cell adhesion. Subtypes: GO:0160018